{
  "gene": "UniProtKB:Q8TED9",
  "gene_name": "Actin filament-associated protein 1-like 1",
  "gene_symbol": "AFAP1L1",
  "term_id": "GO:0005829",
  "term_label": "cytosol"
}